{
  "gene": "UniProtKB:Q8WTR4",
  "term_id": "GO:0008889",
  "gene_name": "Glycerophosphodiester phosphodiesterase domain-containing protein 5",
  "term_label": "glycerophosphodiester phosphodiesterase activity",
  "gene_symbol": "GDPD5"
}